{
  "term_label": "nucleus",
  "gene_symbol": "BTG3",
  "term_id": "GO:0005634",
  "gene": "UniProtKB:Q14201",
  "gene_name": "Protein BTG3"
}